{
  "gene_symbol": "SSTR2",
  "term_id": "GO:0042923",
  "term_label": "neuropeptide binding",
  "gene_name": "Somatostatin receptor type 2",
  "gene": "UniProtKB:P30874"
}